{
  "gene": "UniProtKB:Q96RJ3",
  "term_id": "GO:0042102",
  "gene_name": "Tumor necrosis factor receptor superfamily member 13C",
  "term_label": "positive regulation of T cell proliferation",
  "gene_symbol": "TNFRSF13C"
}